{
  "gene": "UniProtKB:Q07864",
  "term_id": "GO:0000278",
  "gene_symbol": "POLE",
  "term_label": "mitotic cell cycle",
  "gene_name": "DNA polymerase epsilon catalytic subunit A"
}